response to nutrient [GO:0007584] (biological process) Definition: Any process that results in a change in state or activity of a cell or an organism (in terms of movement, secretion, enzyme production, gene expression, etc.) as a result of a nutrient stimulus. Also known as: response to nutrients, nutritional response pathway Subtypes: detection of nutrient [GO:0009594], GO:0031670, GO:0033273 Sources: GOC:go_curators Relationships: is a type of response to nutrient levels [GO:0031667]; is a type of response to chemical [GO:0042221]